{
  "gene_name": "Protein wntless homolog",
  "gene_symbol": "WLS",
  "gene": "UniProtKB:Q5T9L3",
  "term_label": "Wnt protein secretion",
  "term_id": "GO:0061355"
}